embryonic skeletal system development [GO:0048706] (biological process) References: PMID:16049113 Sources: GOC:dph, GOC:dsf, GOC:jid, GOC:tb Definition: The process, occurring during the embryonic phase, whose specific outcome is the progression of the skeleton over time, from its formation to the mature structure. Subtypes: embryonic skeletal joint development [GO:0072498] Also known as: embryonic skeletal development Relationships: is a type of skeletal system development [GO:0001501]; is part of GO:0043009